{
  "gene_name": "Sex comb on midleg-like protein 4",
  "gene": "UniProtKB:Q8N228",
  "gene_symbol": "SCML4",
  "term_label": "histone binding",
  "term_id": "GO:0042393"
}